nicotinate nucleotide biosynthetic process [GO:0019357] (biological process) Sources: GOC:go_curators Also known as: nicotinate nucleotide anabolism, nicotinate nucleotide biosynthesis, nicotinate nucleotide formation, nicotinate nucleotide synthesis Subtypes: nicotinate nucleotide biosynthetic process from tryptophan [GO:0019356], nicotinate nucleotide salvage [GO:0019358] Relationships: is a type of pyridine nucleotide biosynthetic process [GO:0019363] Definition: The chemical reactions and pathways resulting in the formation of nicotinamide nucleotides, any nucleotide that contains combined nicotinate (pyridine 3-carboxylic acid).